{
  "gene_name": "PRKCA-binding protein",
  "term_id": "GO:0002092",
  "term_label": "positive regulation of receptor internalization",
  "gene": "UniProtKB:Q9NRD5",
  "gene_symbol": "PICK1"
}